negative regulation of Wnt signaling pathway involved in heart development [GO:0003308] (biological process) Definition: Any process that decreases the rate, frequency, or extent of the series of molecular signals initiated by binding of Wnt protein to a frizzled family receptor on the surface of the target cell, resulting a change in cell state that contributes to the progression of the heart over time. Also known as: negative regulation of Wnt receptor signaling pathway involved in heart development, negative regulation of Wnt receptor signalling pathway involved in heart development, negative regulation of Wnt-activated signaling pathway involved in heart development Sources: GOC:mtg_heart Relationships: is a type of GO:0003307; is a type of negative regulation of Wnt signaling pathway [GO:0030178]; is a type of negative regulation of developmental process [GO:0051093]; is a type of negative regulation of multicellular organismal process [GO:0051241]; negatively regulates Wnt signaling pathway involved in heart development [GO:0003306]